RNA exonuclease activity [GO:0004532] (molecular function) Regulation: positively regulated by exoribonuclease activator activity [GO:0044692] Definition: Catalysis of the sequential cleavage of mononucleotides from a free 5' or 3' terminus of an RNA molecule. Relationships: is_a exonuclease activity [GO:0004527]; is a type of RNA nuclease activity [GO:0004540] Sources: GOC:mah, ISBN:0198547684 Also known as: exoribonuclease activity Subtypes: GO:0016896, 5'-hydroxyl dinucleotide hydrolase activity [GO:0140432]